{
  "gene": "UniProtKB:Q9UN75",
  "gene_symbol": "PCDHA12",
  "term_id": "GO:0050839",
  "term_label": "cell adhesion molecule binding",
  "gene_name": "Protocadherin alpha-12"
}